{
  "gene_name": "Leucine-rich repeats and immunoglobulin-like domains protein 3",
  "gene_symbol": "LRIG3",
  "term_label": "sensory perception of sound",
  "term_id": "GO:0007605",
  "gene": "UniProtKB:Q6UXM1"
}